Golgi medial cisterna [GO:0005797] (cellular component) Also known as: Golgi apparatus medial cisterna Sources: ISBN:0815316194 Definition: The middle Golgi cisterna (or cisternae). Relationships: is a type of Golgi cisterna [GO:0031985]